{
  "term_label": "positive regulation of macrophage differentiation",
  "gene_symbol": "CSF1",
  "gene": "UniProtKB:P09603",
  "term_id": "GO:0045651",
  "gene_name": "Macrophage colony-stimulating factor 1"
}